{
  "gene_name": "MAM and LDL-receptor class A domain-containing protein 1",
  "gene_symbol": "MALRD1",
  "term_id": "GO:0005794",
  "term_label": "Golgi apparatus",
  "gene": "UniProtKB:Q5VYJ5"
}